{
  "term_id": "UNKNOWN:0001",
  "gene": "UniProtKB:Q8N485",
  "gene_symbol": "LIX1",
  "term_label": "Unknown molecular function",
  "gene_name": "Protein limb expression 1 homolog"
}